{
  "gene_name": "Zinc finger protein 292",
  "term_id": "GO:0006357",
  "term_label": "regulation of transcription by RNA polymerase II",
  "gene_symbol": "ZNF292",
  "gene": "UniProtKB:O60281"
}